{
  "gene": "UniProtKB:Q9Y4J8",
  "term_label": "synapse",
  "gene_symbol": "DTNA",
  "gene_name": "Dystrobrevin alpha",
  "term_id": "GO:0045202"
}